{
  "gene": "UniProtKB:O94888",
  "gene_name": "UBX domain-containing protein 7",
  "term_id": "GO:0043130",
  "term_label": "ubiquitin binding",
  "gene_symbol": "UBXN7"
}